{
  "gene_name": "Coiled-coil domain-containing protein 73",
  "gene_symbol": "CCDC73",
  "term_label": "Unknown biological process",
  "term_id": "UNKNOWN:0002",
  "gene": "UniProtKB:Q6ZRK6"
}